{
  "term_label": "ribosome biogenesis",
  "term_id": "GO:0042254",
  "gene_name": "Cullin-4A",
  "gene": "UniProtKB:Q13619",
  "gene_symbol": "CUL4A"
}